cytosolic small ribosomal subunit assembly [GO:0180025] (biological process) References: PMID:30467428 Definition: The aggregation, arrangement and bonding together of a set of components to form a cytosolic small ribosomal subunit. Relationships: is a type of ribosomal small subunit assembly [GO:0000028]; is part of GO:0042256